histone H3K4 acetyltransferase activity [GO:0044016] (molecular function) Definition: Catalysis of the reaction: acetyl-CoA + histone H3 L-lysine (position 4) = CoA + histone H3 N6-acetyl-L-lysine (position 4). References: PMID:18552846 Also known as: histone H3-K4 acetyltransferase activity, histone acetylase activity (H3-K4 specific), histone acetyltransferase activity (H3-K4 specific), histone lysine N-acetyltransferase activity (H3-K4 specific) Note: Comment: Note that the residue position corresponds to the canonical human H3 histone (UniProtKB:P84243); this residue is conserved across all eukaryotes. Residue 1 is the first residue following removal of the initiating Methionine (Met). Note that each histone is encoded by multiple genes, and sequences may vary across different genes within an organism. Relationships: is a type of histone H3 acetyltransferase activity [GO:0010484]